{
  "gene_name": "Corticotropin-releasing factor-binding protein",
  "gene_symbol": "CRHBP",
  "term_label": "negative regulation of corticotropin secretion",
  "term_id": "GO:0051460",
  "gene": "UniProtKB:P24387"
}